{
  "term_id": "GO:0005886",
  "term_label": "plasma membrane",
  "gene_symbol": "MYOT",
  "gene_name": "Myotilin",
  "gene": "UniProtKB:Q9UBF9"
}